positive regulation of protein localization to cell-cell junction [GO:0150107] (biological process) Definition: Any process that activates or increases the frequency, rate or extent of protein localization to cell-cell junction. Subtypes: positive regulation of protein localization to adherens junction [GO:1904704] References: PMID:26706435 Sources: GOC:aruk, GOC:bc Relationships: is a type of regulation of protein localization to cell-cell junction [GO:0150106]; is a type of positive regulation of protein localization [GO:1903829]; positively regulates protein localization to cell-cell junction [GO:0150105]